{
  "term_label": "dynein light intermediate chain binding",
  "gene_symbol": "CCDC88A",
  "gene": "UniProtKB:Q3V6T2",
  "term_id": "GO:0051959",
  "gene_name": "Girdin"
}